D-valine metabolic process [GO:1902114] (biological process) Definition: The chemical reactions and pathways involving D-valine. Also known as: D-valine metabolism References: PMID:23085840 Sources: GOC:TermGenie Relationships: is a type of GO:0006573; is a type of GO:0046416 Subtypes: GO:1902079